{
  "gene_name": "Serine_threonine-protein kinase PLK2",
  "gene": "UniProtKB:Q9NYY3",
  "term_id": "GO:0005737",
  "gene_symbol": "PLK2",
  "term_label": "cytoplasm"
}